cytosol [GO:0005829] (cellular component) Definition: The part of the cytoplasm that does not contain organelles but which does contain other particulate matter, such as protein complexes. Sources: GOC:hjd, GOC:jl Subtypes: GO:0099522 Relationships: is a type of cellular anatomical structure [GO:0110165]; is part of cytoplasm [GO:0005737]